{
  "term_id": "GO:0006887",
  "gene_symbol": "WASH2P",
  "term_label": "exocytosis",
  "gene_name": "WAS protein family homolog 2",
  "gene": "UniProtKB:Q6VEQ5"
}